{
  "term_label": "endomembrane system",
  "gene": "UniProtKB:O75558",
  "gene_name": "Syntaxin-11",
  "gene_symbol": "STX11",
  "term_id": "GO:0012505"
}